{
  "term_label": "Unknown molecular function",
  "gene_name": "Putative zinc finger protein 826",
  "gene_symbol": "ZNF826P",
  "gene": "UniProtKB:Q6ZT77",
  "term_id": "UNKNOWN:0001"
}